{
  "term_label": "antibacterial humoral response",
  "term_id": "GO:0019731",
  "gene_name": "Lactotransferrin",
  "gene": "UniProtKB:P02788",
  "gene_symbol": "LTF"
}